{
  "gene": "UniProtKB:P36537",
  "gene_name": "UDP-glucuronosyltransferase 2B10",
  "gene_symbol": "UGT2B10",
  "term_id": "GO:0008194",
  "term_label": "UDP-glycosyltransferase activity"
}